cardiac fibroblast cell differentiation [GO:0060935] (biological process) Subtypes: epicardium-derived cardiac fibroblast cell differentiation [GO:0060938], GO:0060942 Relationships: is a type of cardiocyte differentiation [GO:0035051] Sources: GOC:mtg_heart Definition: The process in which a relatively unspecialized cell acquires the specialized structural and/or functional features of a cardiac fibroblast. A cardiac fibroblast is a connective tissue cell in the heart which secretes an extracellular matrix rich in collagen and other macromolecules.